protein localization to cell division site [GO:0072741] (biological process) Definition: A cellular protein localization process in which a protein is transported to, or maintained at, the site of cell division. Relationships: is a type of intracellular protein localization [GO:0008104] Regulation: regulated by GO:1901900 Subtypes: protein localization to medial cortex [GO:0071574], protein localization to cell division site after cytokinesis [GO:0098841], GO:1902432, GO:1902575, protein localization to cell division site involved in cell separation after cytokinesis [GO:1904652], GO:1904759, GO:1905345, protein localization to actomyosin contractile ring [GO:1990179] References: PMID:19756689 Sources: GOC:mah Also known as: protein localisation to cell division site